corticospinal neuron axon decussation [GO:0021973] (biological process) Definition: The process in which the migration of an axon growth cone of a pyramidal cell that is part of the corticospinal tract is directed to cross the midline to the contralateral side. References: PMID:9878731 Sources: GOC:cls, GOC:dgh, GOC:dph, GOC:jid, GO_REF:0000021 Relationships: is a type of axon midline choice point recognition [GO:0016199]; is part of corticospinal neuron axon guidance [GO:0021966]